{
  "gene_symbol": "CYSLTR1",
  "gene_name": "Cysteinyl leukotriene receptor 1",
  "term_id": "GO:0005886",
  "term_label": "plasma membrane",
  "gene": "UniProtKB:Q9Y271"
}